{
  "gene": "UniProtKB:Q5T7W0",
  "term_id": "UNKNOWN:0003",
  "term_label": "Unknown cellular component",
  "gene_name": "Zinc finger protein 618",
  "gene_symbol": "ZNF618"
}